regulation of protein homooligomerization [GO:0032462] (biological process) Sources: GOC:mah Definition: Any process that modulates the frequency, rate or extent of protein homooligomerization. Relationships: is_a regulation of protein oligomerization [GO:0032459]; regulates protein homooligomerization [GO:0051260] Subtypes: GO:0032463, positive regulation of protein homooligomerization [GO:0032464], regulation of protein homotetramerization [GO:1901093]